action potential initiation [GO:0099610] (biological process) Definition: The initiating cycle of an action potential. In vertebrate neurons this typically occurs at an axon hillock. Not all initiated axon potentials propagate. References: PMID:19439602 Sources: ISBN:978-0071390118 Also known as: action potential firing, action potential triggering Relationships: is a type of GO:0001508